{
  "gene_name": "Amine oxidase [flavin-containing] B",
  "gene": "UniProtKB:P27338",
  "term_label": "monoamine oxidase activity",
  "gene_symbol": "MAOB",
  "term_id": "GO:0097621"
}